dinucleotide insertion or deletion binding [GO:0032139] (MF) Sources: GOC:vk Also known as: dinucleotide insertion binding Subtypes: dinucleotide repeat insertion binding [GO:0032181] Definition: Binding to a double-stranded DNA region containing a dinucleotide insertion or deletion. Relationships: is_a DNA insertion or deletion binding [GO:0032135]